{
  "gene_symbol": "TRPM4",
  "gene": "UniProtKB:Q8TD43",
  "term_id": "GO:0098655",
  "gene_name": "Transient receptor potential cation channel subfamily M member 4",
  "term_label": "monoatomic cation transmembrane transport"
}